{
  "gene": "UniProtKB:Q8ND71",
  "gene_symbol": "GIMAP8",
  "term_id": "GO:0003924",
  "term_label": "GTPase activity",
  "gene_name": "GTPase IMAP family member 8"
}